ionotropic glutamate receptor complex [GO:0008328] (cellular component) Definition: A multimeric assembly of four or five subunits which form a structure with an extracellular N-terminus and a large loop that together form the ligand binding domain. The C-terminus is intracellular. The ionotropic glutamate receptor complex itself acts as a ligand-gated ion channel; on binding glutamate, charged ions pass through a channel in the center of the receptor complex. Relationships: is a type of monoatomic ion channel complex [GO:0034702]; is a type of GO:0098878 Subtypes: NMDA selective glutamate receptor complex [GO:0017146], AMPA glutamate receptor complex [GO:0032281], kainate selective glutamate receptor complex [GO:0032983] References: PMID:20716669, PMID:34753794